{
  "term_id": "GO:0043495",
  "term_label": "protein-membrane adaptor activity",
  "gene": "UniProtKB:Q99828",
  "gene_symbol": "CIB1",
  "gene_name": "Calcium and integrin-binding protein 1"
}